{
  "gene_name": "Receptor-transporting protein 5",
  "term_label": "Unknown cellular component",
  "gene": "UniProtKB:Q14D33",
  "gene_symbol": "RTP5",
  "term_id": "UNKNOWN:0003"
}